regulation of horizontal cell localization [GO:1902872] (biological process) Also known as: regulation of horizontal cell localisation, regulation of horizontal cell positioning, regulation of laminar positioning of retinal horizontal cell, regulation of retinal horizontal cell positioning Subtypes: negative regulation of horizontal cell localization [GO:1902873], positive regulation of horizontal cell localization [GO:1902874] Relationships: is a type of regulation of localization [GO:0032879]; is a type of regulation of cellular process [GO:0050794]; regulates horizontal cell localization [GO:0035852] References: PMID:16872597 Sources: GOC:TermGenie, GOC:mr, GO_REF:0000058 Definition: Any process that modulates the frequency, rate or extent of horizontal cell localization.